{
  "gene_symbol": "TJP3",
  "term_id": "GO:1905605",
  "gene_name": "Tight junction protein ZO-3",
  "term_label": "positive regulation of blood-brain barrier permeability",
  "gene": "UniProtKB:O95049"
}